negative regulation of cardiolipin metabolic process [GO:1900209] (biological process) Relationships: is a type of regulation of cardiolipin metabolic process [GO:1900208]; is a type of negative regulation of phospholipid metabolic process [GO:1903726]; negatively regulates cardiolipin metabolic process [GO:0032048] Sources: GOC:TermGenie Definition: Any process that stops, prevents or reduces the frequency, rate or extent of cardiolipin metabolic process. Also known as: down regulation of cardiolipin metabolic process, down regulation of cardiolipin metabolism, down-regulation of cardiolipin metabolic process, down-regulation of cardiolipin metabolism, downregulation of cardiolipin metabolic process, downregulation of cardiolipin metabolism, inhibition of cardiolipin metabolism, negative regulation of cardiolipin metabolism, inhibition of cardiolipin metabolic process, down regulation of diphosphatidylglycerol metabolic process, down regulation of diphosphatidylglycerol metabolism, down-regulation of diphosphatidylglycerol metabolic process, down-regulation of diphosphatidylglycerol metabolism, downregulation of diphosphatidylglycerol metabolic process, downregulation of diphosphatidylglycerol metabolism, inhibition of diphosphatidylglycerol metabolic process, inhibition of diphosphatidylglycerol metabolism, negative regulation of diphosphatidylglycerol metabolic process, negative regulation of diphosphatidylglycerol metabolism